{
  "gene": "UniProtKB:P60484",
  "term_id": "GO:0048870",
  "gene_symbol": "PTEN",
  "gene_name": "Phosphatidylinositol 3,4,5-trisphosphate 3-phosphatase and dual-specificity protein phosphatase PTEN",
  "term_label": "cell motility"
}